{
  "gene_name": "Transient receptor potential cation channel subfamily V member 1",
  "gene": "UniProtKB:Q8NER1",
  "term_id": "GO:0098703",
  "gene_symbol": "TRPV1",
  "term_label": "calcium ion import across plasma membrane"
}